{
  "gene_symbol": "POU3F1",
  "term_label": "regulation of transcription by RNA polymerase II",
  "gene_name": "POU domain, class 3, transcription factor 1",
  "term_id": "GO:0006357",
  "gene": "UniProtKB:Q03052"
}